{
  "gene_name": "Pre-mRNA-processing factor 39",
  "term_label": "U1 snRNP",
  "gene_symbol": "PRPF39",
  "term_id": "GO:0005685",
  "gene": "UniProtKB:Q86UA1"
}